{
  "gene_symbol": "SUSD1",
  "term_id": "UNKNOWN:0001",
  "term_label": "Unknown molecular function",
  "gene_name": "Sushi domain-containing protein 1",
  "gene": "UniProtKB:Q6UWL2"
}